{
  "term_label": "Unknown biological process",
  "gene_symbol": "ZNF22-AS1",
  "gene": "UniProtKB:Q5T742",
  "gene_name": "Uncharacterized protein ZNF22-AS1",
  "term_id": "UNKNOWN:0002"
}